{
  "gene_name": "FAST kinase domain-containing protein 4",
  "term_id": "GO:0035770",
  "gene": "UniProtKB:Q969Z0",
  "gene_symbol": "TBRG4",
  "term_label": "ribonucleoprotein granule"
}